{
  "gene": "UniProtKB:P68036",
  "term_label": "ubiquitin conjugating enzyme activity",
  "gene_symbol": "UBE2L3",
  "term_id": "GO:0061631",
  "gene_name": "Ubiquitin-conjugating enzyme E2 L3"
}